{
  "gene_symbol": "TUBB",
  "term_label": "GTP binding",
  "gene": "UniProtKB:P07437",
  "term_id": "GO:0005525",
  "gene_name": "Tubulin beta chain"
}